{
  "term_label": "Unknown biological process",
  "gene": "UniProtKB:Q6ZV29",
  "gene_name": "Patatin-like phospholipase domain-containing protein 7",
  "term_id": "UNKNOWN:0002",
  "gene_symbol": "PNPLA7"
}